{
  "term_label": "positive regulation of fatty acid oxidation",
  "gene_symbol": "KLHL25",
  "term_id": "GO:0046321",
  "gene_name": "Kelch-like protein 25",
  "gene": "UniProtKB:Q9H0H3"
}